{
  "term_id": "GO:0043065",
  "term_label": "positive regulation of apoptotic process",
  "gene": "UniProtKB:Q9UNL4",
  "gene_symbol": "ING4",
  "gene_name": "Inhibitor of growth protein 4"
}